{
  "gene": "UniProtKB:Q9H2E6",
  "term_label": "positive regulation of neuron migration",
  "gene_symbol": "SEMA6A",
  "gene_name": "Semaphorin-6A",
  "term_id": "GO:2001224"
}